{
  "term_label": "membrane",
  "gene": "UniProtKB:Q8NEB5",
  "gene_symbol": "PLPP5",
  "term_id": "GO:0016020",
  "gene_name": "Phospholipid phosphatase 5"
}